{
  "gene_symbol": "HPCA",
  "term_label": "calcium ion binding",
  "gene_name": "Neuron-specific calcium-binding protein hippocalcin",
  "term_id": "GO:0005509",
  "gene": "UniProtKB:P84074"
}